{
  "term_label": "Unknown molecular function",
  "term_id": "UNKNOWN:0001",
  "gene_symbol": "UBAP2",
  "gene": "UniProtKB:Q5T6F2",
  "gene_name": "Ubiquitin-associated protein 2"
}